{
  "term_id": "GO:0010494",
  "gene": "UniProtKB:P11940",
  "gene_symbol": "PABPC1",
  "term_label": "cytoplasmic stress granule",
  "gene_name": "Polyadenylate-binding protein 1"
}